{
  "gene": "UniProtKB:Q6PIW4",
  "term_label": "nucleus",
  "term_id": "GO:0005634",
  "gene_name": "Fidgetin-like protein 1",
  "gene_symbol": "FIGNL1"
}